nicotinamide riboside transmembrane transporter activity [GO:0034257] (molecular function) Definition: Enables the transfer of nicotinamide riboside, which is a pyridine-3-carboxamide covalently bonded to a ribose sugar, from one side of a membrane to the other. Relationships: is a type of nucleoside transmembrane transporter activity [GO:0005337]; is part of GO:0034258 Sources: GOC:se